{
  "term_id": "GO:0007015",
  "term_label": "actin filament organization",
  "gene": "UniProtKB:O43795",
  "gene_name": "Unconventional myosin-Ib",
  "gene_symbol": "MYO1B"
}